{
  "gene_symbol": "IL2RG",
  "gene": "UniProtKB:P31785",
  "gene_name": "Cytokine receptor common subunit gamma",
  "term_id": "GO:0004896",
  "term_label": "cytokine receptor activity"
}